regulation of inflammatory response [GO:0050727] (biological process) Subtypes: regulation of acute inflammatory response [GO:0002673], regulation of chronic inflammatory response [GO:0002676], GO:0002861, GO:0050728, GO:0050729, GO:0060264, GO:0106014, regulation of neuroinflammatory response [GO:0150077], regulation of histamine secretion by mast cell [GO:1903593] Sources: GOC:ai Relationships: is a type of GO:0031347; is a type of regulation of response to external stimulus [GO:0032101]; regulates inflammatory response [GO:0006954] Definition: Any process that modulates the frequency, rate or extent of the inflammatory response, the immediate defensive reaction (by vertebrate tissue) to infection or injury caused by chemical or physical agents.